{
  "term_id": "GO:0071013",
  "gene_name": "U6 snRNA-associated Sm-like protein LSm2",
  "gene": "UniProtKB:Q9Y333",
  "term_label": "catalytic step 2 spliceosome",
  "gene_symbol": "LSM2"
}